{
  "term_id": "UNKNOWN:0001",
  "gene_name": "Ly6_PLAUR domain-containing protein 8",
  "gene_symbol": "LYPD8",
  "gene": "UniProtKB:Q6UX82",
  "term_label": "Unknown molecular function"
}